{
  "term_label": "Golgi cisterna",
  "gene": "UniProtKB:Q9BZG1",
  "gene_name": "Ras-related protein Rab-34",
  "gene_symbol": "RAB34",
  "term_id": "GO:0031985"
}